{
  "gene_name": "Tumor necrosis factor ligand superfamily member 4",
  "gene": "UniProtKB:P23510",
  "gene_symbol": "TNFSF4",
  "term_label": "positive regulation of T cell proliferation",
  "term_id": "GO:0042102"
}